{
  "gene": "UniProtKB:Q53TS8",
  "term_id": "UNKNOWN:0003",
  "term_label": "Unknown cellular component",
  "gene_symbol": "C2CD6",
  "gene_name": "Cation channel sperm-associated targeting subunit tau"
}